positive regulation of mitotic cell cycle DNA replication [GO:1903465] (biological process) Relationships: is_a GO:0010571; is_a GO:0045931; is a type of regulation of mitotic cell cycle DNA replication [GO:1903463]; positively regulates mitotic DNA replication [GO:1902969] References: PMID:1234 Sources: GOC:TermGenie, GOC:mtg_cell_cycle, GO_REF:0000058 Definition: Any process that activates or increases the frequency, rate or extent of mitotic cell cycle DNA replication. Subtypes: GO:1903468 Also known as: positive regulation of DNA replication involved in S phase involved in mitotic cell cycle, positive regulation of DNA replication involved in S-phase involved in mitotic cell cycle, positive regulation of mitotic nuclear cell cycle DNA replication, up regulation of DNA replication involved in S phase involved in mitotic cell cycle, up regulation of DNA replication involved in S-phase involved in mitotic cell cycle, up regulation of mitotic cell cycle DNA replication, up regulation of mitotic nuclear cell cycle DNA replication, up-regulation of DNA replication involved in S phase involved in mitotic cell cycle, up-regulation of DNA replication involved in S-phase involved in mitotic cell cycle, up-regulation of mitotic cell cycle DNA replication, up-regulation of mitotic nuclear cell cycle DNA replication, upregulation of DNA replication involved in S phase involved in mitotic cell cycle, upregulation of DNA replication involved in S-phase involved in mitotic cell cycle, upregulation of mitotic cell cycle DNA replication, upregulation of mitotic nuclear cell cycle DNA replication, activation of DNA replication involved in S phase involved in mitotic cell cycle, activation of DNA replication involved in S-phase involved in mitotic cell cycle, activation of mitotic cell cycle DNA replication, activation of mitotic nuclear cell cycle DNA replication, activation of DNA replication during S phase involved in mitotic cell cycle, activation of nuclear cell cycle DNA replication involved in mitotic cell cycle, positive regulation of DNA replication during S phase involved in mitotic cell cycle, positive regulation of nuclear cell cycle DNA replication involved in mitotic cell cycle, up regulation of DNA replication during S phase involved in mitotic cell cycle, up regulation of nuclear cell cycle DNA replication involved in mitotic cell cycle, up-regulation of DNA replication during S phase involved in mitotic cell cycle, up-regulation of nuclear cell cycle DNA replication involved in mitotic cell cycle, upregulation of DNA replication during S phase involved in mitotic cell cycle, upregulation of nuclear cell cycle DNA replication involved in mitotic cell cycle